{
  "gene": "UniProtKB:Q92914",
  "gene_symbol": "FGF11",
  "gene_name": "Fibroblast growth factor 11",
  "term_id": "GO:0022008",
  "term_label": "neurogenesis"
}